{
  "gene_symbol": "EVC2",
  "gene": "UniProtKB:Q86UK5",
  "term_label": "plasma membrane protein complex",
  "gene_name": "Limbin",
  "term_id": "GO:0098797"
}